{
  "term_id": "GO:0045944",
  "gene_symbol": "SOX2",
  "gene_name": "Transcription factor SOX-2",
  "term_label": "positive regulation of transcription by RNA polymerase II",
  "gene": "UniProtKB:P48431"
}